{
  "gene_symbol": "VPS41",
  "term_label": "HOPS complex",
  "gene": "UniProtKB:P49754",
  "gene_name": "Vacuolar protein sorting-associated protein 41 homolog",
  "term_id": "GO:0030897"
}